{
  "term_label": "plasma membrane",
  "term_id": "GO:0005886",
  "gene_symbol": "SIRPB2",
  "gene_name": "Signal-regulatory protein beta-2",
  "gene": "UniProtKB:Q5JXA9"
}